anaerobic 2,4,6-trinitrotoluene catabolic process [GO:0046258] (biological process) Relationships: is a type of 2,4,6-trinitrotoluene catabolic process [GO:0046256] Also known as: anaerobic 2,4,6-trinitrotoluene breakdown, anaerobic 2,4,6-trinitrotoluene catabolism, anaerobic 2,4,6-trinitrotoluene degradation Definition: The chemical reactions and pathways resulting in the breakdown of 2,4,6-trinitrotoluene, 1-methyl-2,4,6-trinitrobenzene, a highly explosive pale yellow crystalline solid, in the absence of oxygen. Sources: GOC:ai